hydroxycinnamoyltransferase activity [GO:0050734] (molecular function) Definition: Catalysis of the transfer of a hydroxycinnamoyl group to an acceptor molecule. Subtypes: putrescine N-hydroxycinnamoyltransferase activity [GO:0047174], O-hydroxycinnamoyltransferase activity [GO:0050737] Sources: GOC:ai Relationships: is_a acyltransferase activity, transferring groups other than amino-acyl groups [GO:0016747]